dihydrobiopterin metabolic process [GO:0051066] (biological process) Definition: The chemical reactions and pathways involving a dihydrobiopterin, a reduced pteridine derivative related to folic acid; it acts as an electron carrier in tyrosine biosynthesis and its quinoid form is produced by oxidation of tetrahydrobiopterin in several biological hydroxylation reactions. References: PMID:2557335 Also known as: dihydropterin metabolic process, dihydropterin metabolism, 6,7-dihydrobiopterin metabolic process, 7,8-dihydrobiopterin metabolic process, dihydrobiopterin reduction Relationships: is_a pteridine-containing compound metabolic process [GO:0042558]